{
  "gene_symbol": "TRIM34",
  "gene_name": "E3 ubiquitin-protein ligase TRIM34",
  "term_label": "ubiquitin protein ligase activity",
  "gene": "UniProtKB:Q9BYJ4",
  "term_id": "GO:0061630"
}